{
  "gene_name": "Large ribosomal subunit protein eL43",
  "term_label": "cytosolic large ribosomal subunit",
  "gene_symbol": "RPL37A",
  "gene": "UniProtKB:P61513",
  "term_id": "GO:0022625"
}